monosaccharide biosynthetic process [GO:0046364] (biological process) Definition: The chemical reactions and pathways resulting in the formation of monosaccharides, polyhydric alcohols containing either an aldehyde or a keto group and between three to ten or more carbon atoms. Subtypes: GO:0019294, GO:0019319, pentose biosynthetic process [GO:0019322], L-ascorbic acid biosynthetic process [GO:0019853], tetrose biosynthetic process [GO:0033348], D-galacturonate biosynthetic process [GO:0033482], 2-dehydro-3-deoxy-D-gluconic acid biosynthetic process [GO:1901274], GO:1901803 Sources: ISBN:0198506732 Relationships: is a type of monosaccharide metabolic process [GO:0005996]; is a type of GO:0016051; is a type of small molecule biosynthetic process [GO:0044283] Also known as: monosaccharide anabolism, monosaccharide biosynthesis, monosaccharide formation, monosaccharide synthesis